{
  "term_label": "amino acid transmembrane transport",
  "gene_name": "Putative sodium-coupled neutral amino acid transporter 11",
  "gene": "UniProtKB:Q08AI6",
  "gene_symbol": "SLC38A11",
  "term_id": "GO:0003333"
}